{
  "gene": "UniProtKB:P04040",
  "term_id": "GO:0020037",
  "gene_name": "Catalase",
  "term_label": "heme binding",
  "gene_symbol": "CAT"
}